{
  "gene_symbol": "GAR1",
  "gene": "UniProtKB:Q9NY12",
  "term_label": "box H/ACA snoRNA binding",
  "gene_name": "H_ACA ribonucleoprotein complex subunit 1",
  "term_id": "GO:0034513"
}